3-phosphoinositide-dependent protein kinase binding [GO:0043423] (molecular function) Sources: GOC:jl Relationships: is a type of protein kinase binding [GO:0019901] Also known as: phosphatidylinositol-3-phosphate-dependent protein kinase binding Definition: Binding to a 3-phosphoinositide-dependent protein kinase.